clearance of cells from fusion plate [GO:0060884] (biological process) Subtypes: clearance of cells from fusion plate by apoptotic process [GO:0060885], clearance of cells from fusion plate by epithelial to mesenchymal transition [GO:0060886] Definition: The morphogenetic process in which cells are removed from the inner loop of a semicircular canal. Relationships: is a type of morphogenesis of an epithelium [GO:0002009]; is a type of embryonic morphogenesis [GO:0048598]; is part of semicircular canal morphogenesis [GO:0048752] Sources: GOC:dph, GOC:sdb_2009, GOC:tb